{
  "term_label": "Unknown cellular component",
  "gene_name": "Secernin-1",
  "gene": "UniProtKB:Q12765",
  "gene_symbol": "SCRN1",
  "term_id": "UNKNOWN:0003"
}